maintenance of secretory granule location [GO:0032255] (biological process) Definition: Any process in which a secretory granule is maintained in a specific location within a cell and prevented from moving elsewhere. Subtypes: maintenance of dense core granule location [GO:0032257] Also known as: maintenance of secretory granule localization Sources: GOC:dph, GOC:mah, GOC:tb Relationships: is a type of GO:0051655; is part of GO:0032252